{
  "gene_symbol": "TRAPPC2L",
  "gene": "UniProtKB:Q9UL33",
  "gene_name": "Trafficking protein particle complex subunit 2-like protein",
  "term_id": "GO:0006888",
  "term_label": "endoplasmic reticulum to Golgi vesicle-mediated transport"
}